{
  "gene_name": "Peptide-N(4)-(N-acetyl-beta-glucosaminyl)asparagine amidase",
  "term_id": "GO:0005829",
  "term_label": "cytosol",
  "gene": "UniProtKB:Q96IV0",
  "gene_symbol": "NGLY1"
}